{
  "gene": "UniProtKB:P18433",
  "term_label": "Unknown cellular component",
  "gene_symbol": "PTPRA",
  "gene_name": "Receptor-type tyrosine-protein phosphatase alpha",
  "term_id": "UNKNOWN:0003"
}